negative regulation of nervous system development [GO:0051961] (BP) Relationships: is a type of GO:0051093; is a type of negative regulation of multicellular organismal process [GO:0051241]; is a type of regulation of nervous system development [GO:0051960]; negatively regulates nervous system development [GO:0007399] Also known as: down regulation of nervous system development, down-regulation of nervous system development, downregulation of nervous system development, inhibition of nervous system development Sources: GOC:ai Subtypes: negative regulation of anterior neural cell fate commitment of the neural plate [GO:0022001], negative regulation of neurogenesis [GO:0050768], negative regulation of synapse assembly [GO:0051964] Definition: Any process that stops, prevents, or reduces the frequency, rate or extent of nervous system development, the origin and formation of nervous tissue.